Mre11 complex [GO:0030870] (cellular component) Definition: Trimeric protein complex that possesses endonuclease activity; involved in meiotic recombination, DNA repair and checkpoint signaling. In Saccharomyces cerevisiae, the complex comprises Mre11p, Rad50p, and Xrs2p; complexes identified in other species generally contain proteins orthologous to the Saccharomyces cerevisiae proteins. References: PMID:11988766, PMID:17674145 Sources: GOC:mah, GOC:vw Also known as: MRN complex, MRX complex, RAD50-MRE11-NBN complex, RMX complex, Rad50 complex, Rad50-Rad32-Nbs1 complex Relationships: is a type of GO:0140513